{
  "gene": "UniProtKB:Q13469",
  "term_label": "calcineurin-NFAT signaling cascade",
  "term_id": "GO:0033173",
  "gene_name": "Nuclear factor of activated T-cells, cytoplasmic 2",
  "gene_symbol": "NFATC2"
}